hemocyte migration [GO:0035099] (biological process) Relationships: is a type of GO:0016477; is part of embryonic hemopoiesis [GO:0035162] Definition: The directed movement of a hemocyte within the embryo. Hemocytes are blood cells associated with a hemocoel (the cavity containing most of the major organs of the arthropod body) which are involved in defense and clotting of hemolymph, but not involved in transport of oxygen. In Drosophila, embryonic hemocytes originate from the head mesoderm as a cluster of cells. The cluster splits into two and one group of cells crosses the amnioserosa. Both populations then spread toward the middle of the embryo and then disperse evenly throughout the embryo. Also known as: arthropod blood cell migration, hemocyte cell migration References: PMID:12885551 Sources: GOC:bf, GOC:mtg_sensu